{
  "term_id": "GO:0048743",
  "gene_symbol": "MYF5",
  "gene_name": "Myogenic factor 5",
  "gene": "UniProtKB:P13349",
  "term_label": "positive regulation of skeletal muscle fiber development"
}